{
  "term_label": "DNA-binding transcription factor activity, RNA polymerase II-specific",
  "term_id": "GO:0000981",
  "gene": "UniProtKB:Q92570",
  "gene_name": "Nuclear receptor subfamily 4 group A member 3",
  "gene_symbol": "NR4A3"
}